cellular response to interleukin-15 [GO:0071350] (biological process) Sources: GOC:mah Relationships: is a type of GO:0070672; is_a cellular response to cytokine stimulus [GO:0071345] Definition: Any process that results in a change in state or activity of a cell (in terms of movement, secretion, enzyme production, gene expression, etc.) as a result of an interleukin-15 stimulus. Also known as: cellular response to IL-15